ATP hydrolysis activity [GO:0016887] (molecular function) Definition: Catalysis of the reaction: ATP + H2O = ADP + H+ phosphate. ATP hydrolysis is used in some reactions as an energy source, for example to catalyze a reaction or drive transport against a concentration gradient. Note: Note that this term is meant to specifically represent the ATPase activity of proteins using ATP as a source of energy to drive a reaction. If possible, gene products should also be annotated to a child of 'ATP-dependent activity ; GO:0140657', to capture their overall function. Also known as: ATP hydrolase activity, ATP phosphohydrolase activity, adenosine 5'-triphosphatase activity, adenosine triphosphatase activity, adenosinetriphosphatase activity, ATP monophosphatase activity Sources: RHEA:13065 Relationships: is a type of GO:0017111; is part of ATP-dependent activity [GO:0140657]